{
  "term_label": "negative regulation of exocytosis",
  "gene_name": "Interleukin-1 receptor accessory protein-like 1",
  "term_id": "GO:0045920",
  "gene_symbol": "IL1RAPL1",
  "gene": "UniProtKB:Q9NZN1"
}